positive regulation of aggregate size involved in sorocarp development [GO:0031159] (biological process) Relationships: is a type of regulation of aggregate size involved in sorocarp development [GO:0031157] Definition: Any process that increases the size of the aggregate formed during sorocarp formation. References: PMID:5002049 Sources: GOC:mah, GOC:pg Also known as: up regulation of aggregate size, up-regulation of aggregate size, upregulation of aggregate size, activation of aggregate size, stimulation of aggregate size